{
  "term_id": "UNKNOWN:0003",
  "gene": "UniProtKB:P55000",
  "gene_name": "Secreted Ly-6_uPAR-related protein 1",
  "term_label": "Unknown cellular component",
  "gene_symbol": "SLURP1"
}